{
  "gene_symbol": "KCTD12",
  "term_id": "GO:0008277",
  "term_label": "regulation of G protein-coupled receptor signaling pathway",
  "gene": "UniProtKB:Q96CX2",
  "gene_name": "BTB_POZ domain-containing protein KCTD12"
}